isopentenyl diphosphate biosynthetic process, mevalonate pathway [GO:0019287] (biological process) Subtypes: isopentenyl diphosphate biosynthetic process, mevalonate pathway involved in terpenoid biosynthetic process [GO:0051486] Also known as: Ac-MVA pathway, acetate-mevalonate pathway, isopentenyl diphosphate anabolism, mevalonate pathway, isopentenyl diphosphate biosynthetic process via mevalonate, isopentenyl diphosphate formation, mevalonate pathway, isopentenyl diphosphate synthesis, mevalonate pathway Relationships: is a type of GO:0006084; is_a isopentenyl diphosphate biosynthetic process [GO:0009240] Sources: GOC:go_curators, MetaCyc:PWY-922 Definition: The chemical reactions and pathways resulting in the formation of isopentenyl diphosphate, via the intermediate mevalonate. This pathway converts acetate, in the form of acetyl-CoA, to isopentenyl diphosphate (IPP), the fundamental unit in isoprenoid biosynthesis, through a series of mevalonate intermediates. Regulation: positively regulated by positive regulation of isopentenyl diphosphate biosynthetic process, mevalonate pathway [GO:1900486]; regulated by regulation of isopentenyl diphosphate biosynthetic process, mevalonate pathway [GO:2001210]; negatively regulated by negative regulation of isopentenyl diphosphate biosynthetic process, mevalonate pathway [GO:2001211]